protein storage vacuole lumen [GO:0034495] (cellular component) Relationships: is a type of plant-type vacuole lumen [GO:0000330]; BFO_0000050 protein storage vacuole [GO:0000326] Definition: The volume enclosed by the protein storage vacuole membrane. Sources: GOC:rph